{
  "term_label": "phosphorylase kinase complex",
  "gene_name": "Phosphorylase b kinase regulatory subunit alpha, liver isoform",
  "gene": "UniProtKB:P46019",
  "gene_symbol": "PHKA2",
  "term_id": "GO:0005964"
}